{
  "term_label": "plasma membrane",
  "gene": "UniProtKB:A6NIZ1",
  "gene_symbol": "RAP1BL",
  "term_id": "GO:0005886",
  "gene_name": "Ras-related protein Rap-1b-like protein"
}